{
  "gene": "UniProtKB:Q96NZ1",
  "term_label": "cis-regulatory region sequence-specific DNA binding",
  "gene_symbol": "FOXN4",
  "gene_name": "Forkhead box protein N4",
  "term_id": "GO:0000987"
}